positive regulation of calcium ion transport into cytosol [GO:0010524] (biological process) Definition: Any process that increases the rate of the directed movement of calcium ions into the cytosol of a cell. The cytosol is that part of the cytoplasm that does not contain membranous or particulate subcellular components. Relationships: is a type of positive regulation of cytosolic calcium ion concentration [GO:0007204]; is a type of regulation of calcium ion transport into cytosol [GO:0010522]; is a type of positive regulation of calcium ion transmembrane transport [GO:1904427]; positively regulates calcium ion transport into cytosol [GO:0060402] Sources: GOC:dph, GOC:tb Subtypes: positive regulation of calcium ion transport into cytosol involved in cellular response to calcium ion [GO:1901198], positive regulation of calcium ion transport into cytosol involved in cellular response to salt stress [GO:1901199]